cyanide hydratase activity [GO:0030196] (molecular function) Sources: EC:4.2.1.66, RHEA:21720 Definition: Catalysis of the reaction: formamide = H2O + hydrogen cyanide. Also known as: formamide dehydratase activity, formamide hydro-lyase (cyanide-forming), formamide hydro-lyase activity Relationships: is a type of hydro-lyase activity [GO:0016836]